xylosyltransferase activity [GO:0042285] (molecular function) Relationships: is a type of pentosyltransferase activity [GO:0016763] Definition: Catalysis of the transfer of a xylosyl group to an acceptor molecule, typically another carbohydrate or a lipid. Subtypes: xyloglucan 6-xylosyltransferase activity [GO:0033843], GO:0035252, dolichyl-xylosyl-phosphate-protein xylosyltransferase activity [GO:0047284] Sources: GOC:ai